{
  "gene": "UniProtKB:Q92599",
  "gene_symbol": "SEPTIN8",
  "term_label": "intracellular protein localization",
  "gene_name": "Septin-8",
  "term_id": "GO:0008104"
}